{
  "term_label": "heterochromatin formation",
  "term_id": "GO:0031507",
  "gene_symbol": "CENPA",
  "gene": "UniProtKB:P49450",
  "gene_name": "Histone H3-like centromeric protein A"
}